myofilament [GO:0036379] (cellular component) Also known as: striated muscle filament Sources: Wikipedia:Myofilament Relationships: is a type of cellular anatomical structure [GO:0110165]; is part of myofibril [GO:0030016] Subtypes: striated muscle myosin thick filament [GO:0005863], GO:0005865 Definition: Any of the smallest contractile units of a myofibril (striated muscle fiber).